{
  "gene": "UniProtKB:Q16778",
  "gene_symbol": "H2BC21",
  "term_label": "chromatin organization",
  "gene_name": "Histone H2B type 2-E",
  "term_id": "GO:0006325"
}